homologous recombination [GO:0035825] (biological process) Definition: A DNA recombination process that results in the exchange of an equal amount of genetic material between highly homologous DNA molecules. References: PMID:11139492, PMID:17304215 Sources: GOC:mah Also known as: interchromosomal DNA recombination, interstrand DNA recombination, reciprocal DNA recombination, chromosomal crossover Relationships: is a type of GO:0006310 Subtypes: GO:0035822, reciprocal homologous recombination [GO:0140527]